{
  "term_id": "GO:0021952",
  "gene_symbol": "SPTBN4",
  "term_label": "central nervous system projection neuron axonogenesis",
  "gene": "UniProtKB:Q9H254",
  "gene_name": "Spectrin beta chain, non-erythrocytic 4"
}